{
  "gene": "UniProtKB:P00995",
  "term_label": "Unknown cellular component",
  "gene_symbol": "SPINK1",
  "gene_name": "Serine protease inhibitor Kazal-type 1",
  "term_id": "UNKNOWN:0003"
}